response to cortisone [GO:0051413] (biological process) References: PMID:11276391 Sources: ISBN:0721662544 Subtypes: GO:0071388 Definition: Any process that results in a change in state or activity of a cell or an organism (in terms of movement, secretion, enzyme production, gene expression, etc.) as a result of a cortisone stimulus. Cortisone is a natural glucocorticoid steroid hormone that is metabolically convertible to cortisol. Cortisone is synthesized from cholesterol in the cortex of the adrenal gland under the stimulation of adrenocorticotropin hormone (ACTH). The main physiological effect of cortisone is on carbohydrate metabolism; it can stimulate increased glucose release from the liver, increased liver glycogen synthesis, and decreased utilization of glucose by the tissues. Relationships: is a type of response to glucocorticoid [GO:0051384]; is a type of response to alcohol [GO:0097305]; is a type of response to ketone [GO:1901654] Also known as: response to cortisone stimulus